{
  "term_label": "heart morphogenesis",
  "term_id": "GO:0003007",
  "gene": "UniProtKB:O15178",
  "gene_symbol": "TBXT",
  "gene_name": "T-box transcription factor T"
}